protein post-translational transfer of dolichol-linked oligosaccharide [GO:0180057] (biological process) Definition: A N-linked protein glycosylation process in which the preassembled dolichol-linked oligosaccharide precursor is transfered co-translationally to an asparagine residue within the motif Asn-X-Ser/Thr of the target protein. This is mediated by the OSTB complex. Relationships: is a type of glycoprotein biosynthetic process [GO:0009101]; is part of GO:0006487 Also known as: protein N-linked glycosylation via asparagine, post-translational, protein N-linked glycosylation via asparagine, posttranslational, protein posttranslational transfer of dolichol-linked oligosaccharide References: PMID:19167329